{
  "gene_symbol": "GAS2",
  "term_id": "GO:0051764",
  "gene": "UniProtKB:O43903",
  "gene_name": "Growth arrest-specific protein 2",
  "term_label": "actin crosslink formation"
}